CHOP-ATF3 complex [GO:1990622] (cellular component) References: PMID:8622660 Sources: GOC:PARL, GOC:bf Relationships: is a type of transcription regulator complex [GO:0005667]; is a type of nuclear protein-containing complex [GO:0140513] Definition: A heterodimeric protein complex that is composed of CHOP (C/EBP homology protein, GADD153) and ATF3 (activating transcription factor 3) subunits. Also known as: ATF3-CHOP complex, CHOP-ATF3 heterodimer, CHOP-ATF3 heterodimeric complex, GADD153-ATF3 complex